mesenchymal-epithelial cell signaling [GO:0060638] (biological process) Definition: Any process that mediates the transfer of information from a mesenchymal cell to an epithelial cell where it is received and interpreted. Also known as: mesenchymal-epithelial cell signalling Relationships: is a type of cell-cell signaling [GO:0007267] Sources: GOC:dph Subtypes: mesenchymal-epithelial cell signaling involved in lung development [GO:0060496], positive regulation of mammary placode formation by mesenchymal-epithelial signaling [GO:0060617], GO:0060637, GO:0060639, positive regulation of dentin-containing tooth bud formation by mesenchymal-epithelial signaling [GO:0060640], regulation of branching involved in salivary gland morphogenesis by mesenchymal-epithelial signaling [GO:0060665], mesenchymal-epithelial cell signaling involved in prostate gland development [GO:0060739]